positive regulation of deadenylation-independent decapping of nuclear-transcribed mRNA [GO:1901835] (biological process) Also known as: activation of deadenylylation-independent decapping, positive regulation of deadenylylation-independent decapping, up regulation of deadenylation-independent decapping of nuclear-transcribed mRNA, up regulation of deadenylylation-independent decapping, up-regulation of deadenylation-independent decapping of nuclear-transcribed mRNA, up-regulation of deadenylylation-independent decapping, upregulation of deadenylation-independent decapping of nuclear-transcribed mRNA, upregulation of deadenylylation-independent decapping, activation of deadenylation-independent decapping of nuclear-transcribed mRNA, activation of deadenylation-independent decapping of nuclear mRNA, positive regulation of deadenylation-independent decapping of nuclear mRNA, up regulation of deadenylation-independent decapping of nuclear mRNA, up-regulation of deadenylation-independent decapping of nuclear mRNA, upregulation of deadenylation-independent decapping of nuclear mRNA Definition: Any process that activates or increases the frequency, rate or extent of deadenylation-independent decapping of nuclear-transcribed mRNA. Sources: GOC:TermGenie Relationships: is a type of GO:0061014; is a type of regulation of deadenylation-independent decapping of nuclear-transcribed mRNA [GO:1901834]; positively regulates deadenylation-independent decapping of nuclear-transcribed mRNA [GO:0031087]